{
  "gene_name": "Transcription factor SOX-12",
  "term_id": "GO:0000122",
  "term_label": "negative regulation of transcription by RNA polymerase II",
  "gene": "UniProtKB:O15370",
  "gene_symbol": "SOX12"
}